trans-L-3-hydroxyproline dehydratase activity [GO:0050346] (molecular function) Relationships: is a type of hydro-lyase activity [GO:0016836] Also known as: trans-L-3-hydroxyproline hydro-lyase (Delta1-pyrroline 2-carboxylate-forming), trans-L-3-hydroxyproline hydro-lyase activity Sources: EC:4.2.1.77, RHEA:10320 Definition: Catalysis of the reaction: trans-L-3-hydroxyproline = 1-pyrroline-2-carboxylate + H2O + H+.